{
  "gene": "UniProtKB:Q9NQZ7",
  "term_id": "GO:0004382",
  "term_label": "GDP phosphatase activity",
  "gene_name": "Ectonucleoside triphosphate diphosphohydrolase 7",
  "gene_symbol": "ENTPD7"
}